{
  "term_id": "GO:0005085",
  "term_label": "guanyl-nucleotide exchange factor activity",
  "gene_name": "Myotubularin-related protein 13",
  "gene": "UniProtKB:Q86WG5",
  "gene_symbol": "SBF2"
}